{
  "gene_symbol": "IGSF6",
  "term_label": "Unknown cellular component",
  "gene_name": "Immunoglobulin superfamily member 6",
  "gene": "UniProtKB:O95976",
  "term_id": "UNKNOWN:0003"
}